{
  "gene": "UniProtKB:Q9Y3T9",
  "gene_symbol": "NOC2L",
  "term_label": "nucleolus",
  "gene_name": "Nucleolar complex protein 2 homolog",
  "term_id": "GO:0005730"
}